{
  "term_label": "small GTPase binding",
  "term_id": "GO:0031267",
  "gene": "UniProtKB:Q8WYP3",
  "gene_name": "Ras and Rab interactor 2",
  "gene_symbol": "RIN2"
}